{
  "term_id": "GO:0045143",
  "gene": "UniProtKB:Q562F6",
  "gene_symbol": "SGO2",
  "gene_name": "Shugoshin 2",
  "term_label": "homologous chromosome segregation"
}